proteasome-mediated ubiquitin-dependent protein catabolic process [GO:0043161] (biological process) Also known as: proteasomal pathway, proteasomal ubiquitin-dependent protein breakdown, proteasomal ubiquitin-dependent protein catabolic process, proteasomal ubiquitin-dependent protein catabolism, proteasomal ubiquitin-dependent protein degradation, proteasomal processing, proteasome pathway Sources: GOC:go_curators Definition: The chemical reactions and pathways resulting in the breakdown of a protein or peptide by hydrolysis of its peptide bonds, initiated by the covalent attachment of ubiquitin, and mediated by the proteasome. Relationships: is a type of ubiquitin-dependent protein catabolic process [GO:0006511]; is_a proteasomal protein catabolic process [GO:0010498] Regulation: regulated by regulation of proteasomal ubiquitin-dependent protein catabolic process [GO:0032434]; negatively regulated by negative regulation of proteasomal ubiquitin-dependent protein catabolic process [GO:0032435]; positively regulated by GO:0032436 Subtypes: negative regulation of transcription by transcription factor catabolism [GO:0010620], GO:0031145, SCF-dependent proteasomal ubiquitin-dependent protein catabolic process [GO:0031146], ubiquitin-dependent protein catabolic process via the N-end rule pathway [GO:0071596], cytoplasm protein quality control by the ubiquitin-proteasome system [GO:0071629], GO:0071630, mitochondria-associated ubiquitin-dependent protein catabolic process [GO:0072671], GO:0120174, ubiquitin-dependent protein catabolic process via the C-end degron rule pathway [GO:0140627], ribosome-associated ubiquitin-dependent protein catabolic process [GO:1990116]